{
  "gene_symbol": "PPP1R42",
  "gene_name": "Protein phosphatase 1 regulatory subunit 42",
  "gene": "UniProtKB:Q7Z4L9",
  "term_label": "Unknown biological process",
  "term_id": "UNKNOWN:0002"
}